nitrogen fixation [GO:0009399] (biological process) Relationships: is a type of nitrogen cycle metabolic process [GO:0071941] Definition: The process in which nitrogen is taken from its relatively inert molecular form (N2) in the atmosphere and converted into ammonium, which is more biologically available. References: PMID:32796519, PMID:36344435